{
  "term_id": "GO:0070628",
  "gene_name": "Ubiquitin D",
  "gene": "UniProtKB:O15205",
  "term_label": "proteasome binding",
  "gene_symbol": "UBD"
}